{
  "gene_name": "SCL-interrupting locus protein",
  "term_label": "protein localization to centrosome",
  "gene": "UniProtKB:Q15468",
  "gene_symbol": "STIL",
  "term_id": "GO:0071539"
}